{
  "gene_symbol": "PABPC1L",
  "term_label": "poly(A) binding",
  "gene": "UniProtKB:Q4VXU2",
  "gene_name": "Polyadenylate-binding protein 1-like",
  "term_id": "GO:0008143"
}